{
  "term_id": "GO:0004930",
  "gene": "UniProtKB:Q7Z602",
  "term_label": "G protein-coupled receptor activity",
  "gene_name": "Probable G-protein coupled receptor 141",
  "gene_symbol": "GPR141"
}